{
  "gene_name": "Putative tripartite motif-containing protein 61",
  "term_label": "regulation of gene expression",
  "term_id": "GO:0010468",
  "gene": "UniProtKB:Q5EBN2",
  "gene_symbol": "TRIM61"
}